regulation of angiotensin metabolic process [GO:0060177] (biological process) Definition: Any process that modulates the frequency, rate or extent of the chemical reactions and pathways involving angiotensin. Sources: GOC:dph, GOC:tb Also known as: regulation of angiotensin metabolism Relationships: is a type of regulation of protein metabolic process [GO:0051246]